{
  "term_id": "GO:0090575",
  "gene_symbol": "ASCL1",
  "gene": "UniProtKB:P50553",
  "gene_name": "Achaete-scute homolog 1",
  "term_label": "RNA polymerase II transcription regulator complex"
}